20-aldehyde-leukotriene B4 20-monooxygenase activity [GO:0097259] (molecular function) References: PMID:2549038, PMID:2836406, PMID:9675028 Sources: GOC:mw, RHEA:48672 Relationships: is a type of GO:0004497 Definition: Catalysis of the reaction: 20-oxo-leukotriene B4 + O2 + reduced [NADPH-hemoprotein reductase] = 20-carboxy-leukotriene B4 + 2 H+ + H2O + oxidized [NADPH-hemoprotein reductase].